{
  "term_id": "UNKNOWN:0002",
  "gene_name": "Zinc finger protein 285",
  "gene_symbol": "ZNF285",
  "gene": "UniProtKB:Q96NJ3",
  "term_label": "Unknown biological process"
}